renal filtration cell differentiation [GO:0061318] (biological process) Relationships: is a type of cell differentiation [GO:0030154]; is part of renal system development [GO:0072001] Definition: The process in which a relatively unspecialized cell acquires specialized structural and/or functional features of a renal filtration cell. Renal filtration cells are specialized cells of the renal system that filter fluids by charge, size or both. Differentiation includes the processes involved in commitment of a cell to a specific fate and its subsequent development to the mature state. Subtypes: nephrocyte differentiation [GO:0061319], podocyte differentiation [GO:0072112] Sources: GOC:dph, GOC:mtg_kidney_jan10